{
  "gene": "UniProtKB:Q96IK5",
  "term_id": "UNKNOWN:0002",
  "gene_name": "Germ cell-less protein-like 1",
  "term_label": "Unknown biological process",
  "gene_symbol": "GMCL1"
}